regulation of establishment of planar polarity involved in neural tube closure [GO:0090178] (biological process) Definition: Any process that modulates the rate, frequency, or extent of the establishment of planar polarity involved in neural tube closure, the coordinated organization of groups of cells in the plane of an epithelium that contributes to the closure of the neural tube. Sources: GOC:ascb_2009, GOC:dph, GOC:tb Relationships: is a type of regulation of establishment of planar polarity [GO:0090175]; regulates establishment of planar polarity involved in neural tube closure [GO:0090177]